{
  "term_id": "GO:0005737",
  "gene": "UniProtKB:P49758",
  "term_label": "cytoplasm",
  "gene_symbol": "RGS6",
  "gene_name": "Regulator of G-protein signaling 6"
}